regulation of cilium assembly [GO:1902017] (biological process) Subtypes: GO:0045724, negative regulation of cilium assembly [GO:1902018], regulation of non-motile cilium assembly [GO:1902855], regulation of motile cilium assembly [GO:1905503] References: PMID:17719545 Sources: GOC:TermGenie, GOC:cilia, GOC:dph Also known as: regulation of ciliogenesis, regulation of cilium biogenesis Definition: Any process that modulates the frequency, rate or extent of cilium assembly. Relationships: is a type of regulation of plasma membrane bounded cell projection assembly [GO:0120032]; is a type of regulation of organelle assembly [GO:1902115]; RO_0002211 cilium assembly [GO:0060271]